antipodal cell degeneration [GO:0055045] (biological process) Relationships: is a type of programmed cell death involved in cell development [GO:0010623]; is part of megagametogenesis [GO:0009561] Sources: GOC:mtg_plant Definition: The process in which the antipodal cells undergo programmed cell death.